{
  "gene": "UniProtKB:Q9H2R5",
  "gene_name": "Kallikrein-15",
  "gene_symbol": "KLK15",
  "term_id": "GO:0004252",
  "term_label": "serine-type endopeptidase activity"
}